{
  "gene_symbol": "FURIN",
  "gene": "UniProtKB:P09958",
  "term_id": "GO:0005802",
  "gene_name": "Furin",
  "term_label": "trans-Golgi network"
}